{
  "gene_name": "Interleukin-23 receptor",
  "term_label": "cytokine binding",
  "gene_symbol": "IL23R",
  "term_id": "GO:0019955",
  "gene": "UniProtKB:Q5VWK5"
}